{
  "gene_name": "Major facilitator superfamily domain-containing protein 6-like",
  "term_id": "GO:0016020",
  "gene": "UniProtKB:Q8IWD5",
  "gene_symbol": "MFSD6L",
  "term_label": "membrane"
}